{
  "gene_name": "Lysosomal-trafficking regulator",
  "term_id": "GO:0005764",
  "gene": "UniProtKB:Q99698",
  "term_label": "lysosome",
  "gene_symbol": "LYST"
}